positive regulation of demethylkotanin biosynthetic process [GO:1900654] (biological process) Definition: Any process that activates or increases the frequency, rate or extent of demethylkotanin biosynthetic process. Sources: GOC:TermGenie, GOC:di Also known as: activation of demethylkotanin anabolism, activation of demethylkotanin biosynthesis, activation of demethylkotanin formation, activation of demethylkotanin synthesis, positive regulation of demethylkotanin anabolism, positive regulation of demethylkotanin biosynthesis, positive regulation of demethylkotanin formation, positive regulation of demethylkotanin synthesis, up regulation of demethylkotanin anabolism, up regulation of demethylkotanin biosynthesis, up regulation of demethylkotanin biosynthetic process, up regulation of demethylkotanin formation, up regulation of demethylkotanin synthesis, up-regulation of demethylkotanin anabolism, up-regulation of demethylkotanin biosynthesis, up-regulation of demethylkotanin biosynthetic process, up-regulation of demethylkotanin formation, up-regulation of demethylkotanin synthesis, upregulation of demethylkotanin anabolism, upregulation of demethylkotanin biosynthesis, upregulation of demethylkotanin biosynthetic process, upregulation of demethylkotanin formation, upregulation of demethylkotanin synthesis, activation of demethylkotanin biosynthetic process Relationships: is a type of positive regulation of secondary metabolite biosynthetic process [GO:1900378]; is a type of GO:1900652; positively regulates GO:1900599